{
  "gene_symbol": "TRGV10",
  "gene_name": "Probable non-functional T cell receptor gamma variable 10",
  "term_id": "UNKNOWN:0001",
  "term_label": "Unknown molecular function",
  "gene": "UniProtKB:A0A0A0MS01"
}